{
  "term_id": "UNKNOWN:0001",
  "term_label": "Unknown molecular function",
  "gene_name": "KN motif and ankyrin repeat domain-containing protein 4",
  "gene_symbol": "KANK4",
  "gene": "UniProtKB:Q5T7N3"
}